{
  "gene": "UniProtKB:Q96SZ4",
  "term_id": "GO:0000978",
  "gene_symbol": "ZSCAN10",
  "term_label": "RNA polymerase II cis-regulatory region sequence-specific DNA binding",
  "gene_name": "Zinc finger and SCAN domain-containing protein 10"
}